{
  "term_label": "Unknown cellular component",
  "gene_symbol": "LRP6",
  "gene_name": "Low-density lipoprotein receptor-related protein 6",
  "term_id": "UNKNOWN:0003",
  "gene": "UniProtKB:O75581"
}